{
  "term_id": "UNKNOWN:0002",
  "term_label": "Unknown biological process",
  "gene": "UniProtKB:Q9NXP7",
  "gene_name": "Gypsy retrotransposon integrase-like protein 1",
  "gene_symbol": "GIN1"
}